{
  "gene": "UniProtKB:P49916",
  "gene_symbol": "LIG3",
  "term_label": "nucleus",
  "term_id": "GO:0005634",
  "gene_name": "DNA ligase 3"
}